positive regulation of transforming growth factor beta1 production [GO:0032914] (biological process) Sources: GOC:mah Also known as: positive regulation of TGF-B1 production, positive regulation of TGFB1 production, up regulation of transforming growth factor-beta1 production, up-regulation of transforming growth factor-beta1 production, upregulation of transforming growth factor-beta1 production, activation of transforming growth factor-beta1 production, stimulation of transforming growth factor-beta1 production Relationships: is a type of regulation of transforming growth factor beta1 production [GO:0032908]; is a type of positive regulation of transforming growth factor beta production [GO:0071636]; positively regulates transforming growth factor beta1 production [GO:0032905] Definition: Any process that activates or increases the frequency, rate, or extent of production of transforming growth factor-beta1.